{
  "gene_name": "Protein C1orf43",
  "gene_symbol": "C1orf43",
  "term_id": "UNKNOWN:0001",
  "term_label": "Unknown molecular function",
  "gene": "UniProtKB:Q9BWL3"
}